cellular response to dimethyl sulfoxide [GO:1904620] (biological process) References: PMID:12873812 Sources: GOC:TermGenie, GO_REF:0000071 Also known as: cellular response to DMSO Relationships: is a type of cellular response to chemical stimulus [GO:0070887]; is a type of GO:1904619 Definition: Any process that results in a change in state or activity of a cell (in terms of movement, secretion, enzyme production, gene expression, etc.) as a result of a dimethyl sulfoxide stimulus.